{
  "term_label": "cellular response to light stimulus",
  "gene_name": "Long-wave-sensitive opsin 1",
  "term_id": "GO:0071482",
  "gene_symbol": "OPN1LW",
  "gene": "UniProtKB:P04000"
}